{
  "gene_name": "Putative uncharacterized protein MRGPRG-AS1",
  "term_id": "UNKNOWN:0003",
  "gene": "UniProtKB:Q2M3A8",
  "gene_symbol": "MRGPRG-AS1",
  "term_label": "Unknown cellular component"
}